{
  "gene": "UniProtKB:Q15554",
  "gene_symbol": "TERF2",
  "term_label": "regulation of telomere maintenance via telomerase",
  "term_id": "GO:0032210",
  "gene_name": "Telomeric repeat-binding factor 2"
}